positive regulation of nitric oxide mediated signal transduction [GO:0010750] (biological process) Sources: GOC:BHF, GOC:dph, GOC:tb Relationships: is a type of regulation of nitric oxide mediated signal transduction [GO:0010749]; is a type of positive regulation of intracellular signal transduction [GO:1902533]; positively regulates nitric oxide mediated signal transduction [GO:0007263] Also known as: positive regulation of nitric oxide-mediated signal transduction Definition: Any process that increases the rate, frequency or extent of nitric oxide mediated signal transduction. Nitric oxide mediated signal transduction is The series of molecular signals mediated by the detection of nitric oxide (NO). Subtypes: positive regulation of nitric oxide-cGMP mediated signal transduction [GO:0141150]